{
  "gene_name": "RNA-binding protein Musashi homolog 1",
  "term_label": "mRNA binding",
  "term_id": "GO:0003729",
  "gene_symbol": "MSI1",
  "gene": "UniProtKB:O43347"
}